{
  "term_id": "GO:0042026",
  "gene_name": "Heat shock cognate 71 kDa protein",
  "gene_symbol": "HSPA8",
  "term_label": "protein refolding",
  "gene": "UniProtKB:P11142"
}